glucuronoxylan catabolic process [GO:2000886] (biological process) Definition: The chemical reactions and pathways resulting in the breakdown of a glucuronoxylan. Sources: GOC:mengo_curators Also known as: glucuronoxylan catabolism Relationships: is a type of glucuronoxylan metabolic process [GO:0010413]; is a type of xylan catabolic process [GO:0045493] Subtypes: glucuronoarabinoxylan catabolic process [GO:2000887] Regulation: regulated by regulation of glucuronoxylan catabolic process [GO:2000915]; negatively regulated by negative regulation of glucuronoxylan catabolic process [GO:2000916]; positively regulated by positive regulation of glucuronoxylan catabolic process [GO:2000917]